extracellular exosome complex [GO:1990563] (cellular component) References: PMID:22660413 Sources: GOC:bhm Definition: A protein complex that is wholly or partially contained within the lumen or membrane of the extracellular vesicular exosome. Subtypes: syndecan-syntenin-ALIX complex [GO:1990562] Also known as: exosome complex, extracellular vesicular exosome complex Note: An example of this is SCD1 in human (UniProt symbol P18827) in PMID:22660413 (inferred from physical interaction). Relationships: is a type of protein-containing complex [GO:0032991]; is part of GO:0070062